{
  "gene_symbol": "NDUFB7",
  "term_label": "respiratory chain complex I",
  "gene_name": "NADH dehydrogenase [ubiquinone] 1 beta subcomplex subunit 7",
  "gene": "UniProtKB:P17568",
  "term_id": "GO:0045271"
}